behavioral response to acetic acid induced pain [GO:0061367] (biological process) Relationships: is a type of behavioral response to chemical pain [GO:0061366] Definition: Any process that results in a change in the behaviour of an organism as a result of an acetic acid pain stimulus. Sources: GOC:dph